{
  "gene": "UniProtKB:Q9HAW8",
  "gene_symbol": "UGT1A10",
  "term_label": "flavone metabolic process",
  "gene_name": "UDP-glucuronosyltransferase 1A10",
  "term_id": "GO:0051552"
}